compound eye corneal lens morphogenesis [GO:0048750] (biological process) Sources: GOC:jid Relationships: is a type of GO:0009653; is part of compound eye morphogenesis [GO:0001745]; is part of GO:0048058 Definition: The process in which the anatomical structures of the compound eye corneal lens are generated and organized.